{
  "gene_name": "Voltage-dependent P_Q-type calcium channel subunit alpha-1A",
  "gene_symbol": "CACNA1A",
  "gene": "UniProtKB:O00555",
  "term_id": "GO:0007268",
  "term_label": "chemical synaptic transmission"
}